negative regulation of branching involved in ureteric bud morphogenesis [GO:0090191] (BP) Definition: Any process that decreases the rate, frequency or extent of branching involved in ureteric bud morphogenesis, the process in which the branching structure of the ureteric bud is generated and organized. The ureteric bud is an epithelial tube that grows out from the metanephric duct. The bud elongates and branches to give rise to the ureter and kidney collecting tubules. Sources: GOC:dph, GOC:tb, GOC:yaf Relationships: is a type of negative regulation of multicellular organismal process [GO:0051241]; is a type of regulation of branching involved in ureteric bud morphogenesis [GO:0090189]; is a type of negative regulation of morphogenesis of an epithelium [GO:1905331]; negatively regulates branching involved in ureteric bud morphogenesis [GO:0001658]